{
  "gene": "UniProtKB:Q9BYX4",
  "gene_symbol": "IFIH1",
  "gene_name": "Interferon-induced helicase C domain-containing protein 1",
  "term_label": "MDA-5 signaling pathway",
  "term_id": "GO:0039530"
}